lipid transfer activity [GO:0120013] (molecular function) References: PMID:20823909, PMID:24220498, PMID:25797198 Sources: GOC:krc Subtypes: glycolipid transfer activity [GO:0017089], phospholipid transfer activity [GO:0120014], sterol transfer activity [GO:0120015], sphingolipid transfer activity [GO:0120016], lipopolysaccharide transfer activity [GO:0140332], diacylglyceride transfer activity [GO:0140337], triglyceride transfer activity [GO:0140344], lipid exchange activity [GO:7770011] Also known as: intermembrane lipid transfer activity, lipid carrier activity Definition: Removes a lipid from a membrane or a monolayer lipid particle, transports it through the aqueous phase while protected in a hydrophobic pocket, and brings it to an acceptor membrane or lipid particle. This results in intermembrane transfer of lipids. Relationships: is a type of lipid transporter activity [GO:0005319]; is part of intermembrane lipid transfer [GO:0120009]